{
  "term_label": "plasma membrane",
  "gene": "UniProtKB:Q8TCU5",
  "gene_symbol": "GRIN3A",
  "gene_name": "Glutamate receptor ionotropic, NMDA 3A",
  "term_id": "GO:0005886"
}